{
  "gene": "UniProtKB:P01880",
  "term_label": "antigen binding",
  "gene_symbol": "IGHD",
  "gene_name": "Immunoglobulin heavy constant delta",
  "term_id": "GO:0003823"
}